{
  "gene_name": "Iroquois-class homeodomain protein IRX-1",
  "gene": "UniProtKB:P78414",
  "term_id": "GO:0000981",
  "term_label": "DNA-binding transcription factor activity, RNA polymerase II-specific",
  "gene_symbol": "IRX1"
}